2'-hydroxybiphenyl-2-sulfinate desulfinase activity [GO:0018740] (molecular function) Also known as: 2'-hydroxybiphenyl-2-sulfinate sulfinolyase activity, 2-(2-hydroxyphenyl)benzenesulphinate hydrolase activity, 2'-hydroxybiphenyl-2-sulfinate sulfohydrolase activity, 2-(2'-hydroxyphenyl)benzenesulfinate desulfinase activity, 2-(2-hydroxyphenyl) benzenesulfinate sulfohydrolase activity, 2-(2-hydroxyphenyl) benzenesulfinate:H2O hydrolase activity, 2-(2-hydroxyphenyl)benzenesulfinate desulfinase activity, 2-(2-hydroxyphenyl)benzenesulfinate hydrolase activity, DszB, HBPSi desulfinase activity, HPBS desulfinase activity, dibenzothiophene desulfurization enzyme B, gene dszB-encoded hydrolase activity Relationships: is a type of hydrolase activity, acting on carbon-sulfur bonds [GO:0046508] Definition: Catalysis of the reaction: 2'-hydroxybiphenyl-2-sulfinate + H2O = biphenyl-2-ol + sulfite. Sources: EC:3.13.1.3, RHEA:12945